{
  "gene_symbol": "CYLD",
  "gene": "UniProtKB:Q9NQC7",
  "term_id": "GO:0061578",
  "gene_name": "Ubiquitin carboxyl-terminal hydrolase CYLD",
  "term_label": "K63-linked deubiquitinase activity"
}